{
  "term_label": "mRNA 3'-end processing by stem-loop binding and cleavage",
  "gene_name": "U7 snRNA-associated Sm-like protein LSm10",
  "gene_symbol": "LSM10",
  "gene": "UniProtKB:Q969L4",
  "term_id": "GO:0006398"
}